{
  "term_label": "lactose catabolic process",
  "term_id": "GO:0005990",
  "gene_name": "Lactase_phlorizin hydrolase",
  "gene": "UniProtKB:P09848",
  "gene_symbol": "LCT"
}